copper ion export [GO:0060003] (biological process) Relationships: is a type of copper ion transmembrane transport [GO:0035434] Sources: GOC:dph Definition: The directed movement of copper ions out of a cell or organelle. Also known as: copper export